{
  "gene_name": "Angiomotin-like protein 1",
  "term_label": "regulation of cell migration",
  "gene_symbol": "AMOTL1",
  "term_id": "GO:0030334",
  "gene": "UniProtKB:Q8IY63"
}